symbiont-mediated perturbation of host small GTPase-mediated signal transduction [GO:0044082] (biological process) Definition: A process in which a symbiont alters or subverts a small GTPase-mediated signal transduction pathway in its host organism. The host is defined as the larger of the organisms involved in a symbiotic interaction. Sources: MITRE:tk Relationships: is a type of regulation of small GTPase mediated signal transduction [GO:0051056]; is a type of GO:0052027 Also known as: modulation by symbiont of host small GTPase mediated signal transduction, modulation of host small GTPase mediated signal transduction by symbiont, perturbation of host small GTPase mediated signal transduction, regulation by symbiont of host small GTPase mediated signal transduction Subtypes: symbiont-mediated perturbation of host Rho small GTPase signal transduction [GO:0044083], symbiont-mediated perturbation of host Rab small GTPase signal transduction [GO:0141127]